UDP-3-O-acyl-N-acetylglucosamine deacetylase activity [GO:0103117] (MF) Sources: GOC:pz, RHEA:67816 Definition: Catalysis of the reaction: a UDP-3-O-[(3R)-3-hydroxyacyl]-N-acetyl-alpha-D-glucosamine + H2O = a UDP-3-O-[(3R)-3-hydroxyacyl]-alpha-D-glucosamine + acetate. Relationships: is a type of hydrolase activity, acting on carbon-nitrogen (but not peptide) bonds, in linear amides [GO:0016811]